{
  "term_id": "UNKNOWN:0001",
  "gene": "UniProtKB:Q9HCM3",
  "term_label": "Unknown molecular function",
  "gene_symbol": "KIAA1549",
  "gene_name": "UPF0606 protein KIAA1549"
}